detection of triacyl bacterial lipopeptide [GO:0042495] (biological process) Definition: The series of events in which a triacylated bacterial lipoprotein stimulus is received by a cell and converted into a molecular signal. Triacylated bacterial lipoproteins are lipopeptides of bacterial origin containing a nonprotein moiety consisting of three acyl groups. References: PMID:12077222, PMID:12524386, PMID:2757794 Sources: GOC:add Also known as: detection of triacylated bacterial lipoprotein, perception of triacylated bacterial lipopeptide, perception of triacylated bacterial lipoprotein Note: Note that bacterial lipopeptides are derived from bacterial lipoproteins, but the two terms are sometimes used interchangeably in the literature. Relationships: is a type of GO:0070340; is a type of response to triacyl bacterial lipopeptide [GO:0071725]